{
  "gene_name": "Akirin-1",
  "gene_symbol": "AKIRIN1",
  "gene": "UniProtKB:Q9H9L7",
  "term_label": "chromatin",
  "term_id": "GO:0000785"
}